{
  "term_id": "GO:0030007",
  "gene_name": "Sodium_potassium-transporting ATPase subunit alpha-3",
  "gene_symbol": "ATP1A3",
  "gene": "UniProtKB:P13637",
  "term_label": "intracellular potassium ion homeostasis"
}